{
  "term_id": "GO:0016020",
  "term_label": "membrane",
  "gene_name": "Synaptojanin-1",
  "gene_symbol": "SYNJ1",
  "gene": "UniProtKB:O43426"
}